{
  "gene_name": "Lithostathine-1-beta",
  "gene_symbol": "REG1B",
  "term_id": "GO:0008083",
  "term_label": "growth factor activity",
  "gene": "UniProtKB:P48304"
}